{
  "gene_symbol": "FASTKD3",
  "gene_name": "FAST kinase domain-containing protein 3, mitochondrial",
  "term_label": "mitochondrial RNA processing",
  "gene": "UniProtKB:Q14CZ7",
  "term_id": "GO:0000963"
}